{
  "gene_name": "Transmembrane O-methyltransferase",
  "term_id": "GO:0042417",
  "gene_symbol": "TOMT",
  "gene": "UniProtKB:Q8WZ04",
  "term_label": "dopamine metabolic process"
}